{
  "gene_name": "Proton-coupled amino acid transporter 1",
  "term_label": "glycine transport",
  "gene": "UniProtKB:Q7Z2H8",
  "gene_symbol": "SLC36A1",
  "term_id": "GO:0015816"
}